negative regulation of hippo signaling [GO:0035331] (biological process) Definition: Any process that stops, prevents, or reduces the frequency, rate or extent of hippo signaling. Also known as: negative regulation of hippo signaling pathway, negative regulation of hippo signaling cascade, negative regulation of hippo signalling cascade Relationships: is a type of regulation of hippo signaling [GO:0035330]; is a type of GO:1902532; negatively regulates hippo signaling [GO:0035329] Sources: GOC:bf